{
  "gene_symbol": "JMY",
  "gene": "UniProtKB:Q8N9B5",
  "term_label": "'de novo' actin filament nucleation",
  "gene_name": "Junction-mediating and -regulatory protein",
  "term_id": "GO:0070060"
}